{
  "term_label": "positive regulation of DNA-templated transcription",
  "gene_symbol": "ILF2",
  "gene_name": "Interleukin enhancer-binding factor 2",
  "term_id": "GO:0045893",
  "gene": "UniProtKB:Q12905"
}